{
  "gene": "UniProtKB:Q6ZUS5",
  "gene_name": "Coiled-coil domain-containing protein 121",
  "gene_symbol": "CCDC121",
  "term_label": "Unknown cellular component",
  "term_id": "UNKNOWN:0003"
}